{
  "term_id": "GO:0006457",
  "gene_symbol": "TCP1",
  "term_label": "protein folding",
  "gene_name": "T-complex protein 1 subunit alpha",
  "gene": "UniProtKB:P17987"
}